{
  "term_label": "positive regulation of type I interferon production",
  "term_id": "GO:0032481",
  "gene": "UniProtKB:Q9NUD5",
  "gene_name": "Zinc finger CCHC domain-containing protein 3",
  "gene_symbol": "ZCCHC3"
}